{
  "gene_symbol": "CCDC191",
  "term_id": "UNKNOWN:0001",
  "gene": "UniProtKB:Q8NCU4",
  "gene_name": "Coiled-coil domain-containing protein 191",
  "term_label": "Unknown molecular function"
}